glycolytic process through glucose-6-phosphate [GO:0061620] (biological process) Subtypes: canonical glycolysis [GO:0061621], glycolytic process through glucose-1-phosphate [GO:0061622], transport-coupled glycolytic process through glucose-6-phosphate [GO:0061633] Relationships: is a type of glycolytic process through fructose-6-phosphate [GO:0061615]; has part glucose-6-phosphate isomerase activity [GO:0004347] Sources: GOC:dph, ISBN:0201090910, ISBN:0879010479 Definition: The chemical reactions and pathways resulting in the breakdown of a carbohydrate into pyruvate, occurring through a glucose-6-phosphate intermediate, with the concomitant production of a small amount of ATP.